ascus lipid droplet [GO:0005633] (cellular component) Definition: Any particle of coalesced lipids in an ascus or ascospore. May include associated proteins. Also known as: ascus lipid particle References: PMID:12702293 Sources: GOC:mah Relationships: is a type of lipid droplet [GO:0005811]